CMP-keto-3-deoxy-D-manno-octulosonic acid biosynthetic process [GO:0033468] (biological process) Definition: The chemical reactions and pathways resulting in the formation of CMP-keto-3-deoxy-D-manno-octulosonic acid, a substance composed of the acidic sugar 3-deoxy-D-manno-octulosonic acid in glycosidic linkage with cytidine monophosphate. Sources: GOC:mah, MetaCyc:PWY-1269 Also known as: CMP-KDO biosynthesis, CMP-KDO biosynthetic process, CMP-keto-3-deoxy-D-manno-octulosonic acid anabolism, CMP-keto-3-deoxy-D-manno-octulosonic acid biosynthesis, CMP-keto-3-deoxy-D-manno-octulosonic acid formation, CMP-keto-3-deoxy-D-manno-octulosonic acid synthesis, CMP-ketodeoxyoctanoate biosynthetic process Relationships: is a type of nucleotide-sugar biosynthetic process [GO:0009226]